{
  "term_id": "GO:0000981",
  "gene_symbol": "FOSB",
  "gene_name": "Protein FosB",
  "gene": "UniProtKB:P53539",
  "term_label": "DNA-binding transcription factor activity, RNA polymerase II-specific"
}